{
  "term_label": "G protein-coupled receptor activity",
  "gene_name": "G-protein coupled receptor 26",
  "term_id": "GO:0004930",
  "gene_symbol": "GPR26",
  "gene": "UniProtKB:Q8NDV2"
}